anther wall tapetum development [GO:0048658] (biological process) Definition: The process whose specific outcome is the progression of the anther wall tapetum over time, from its formation to the mature structure. Also known as: tapetal layer development, tapetum development Sources: GOC:jid, GOC:sm, GOC:tb Relationships: is_a developmental process involved in reproduction [GO:0003006]; is a type of anatomical structure development [GO:0048856]; is part of anther development [GO:0048653]